phytochrome chromophore biosynthetic process [GO:0048543] (biological process) Definition: The chemical reactions and pathways resulting in the formation of the phytochrome chromophore. The phytochrome chromophore is a linear tetrapyrrolic prosthetic group covalently attached to the large soluble protein phytochrome. Light absorption by the phytochrome chromophore triggers photoconversion between two spectrally distinct forms of the photoreceptor: Pr, the red light absorbing form, and Pfr, the far red light absorbing form. References: PMID:2909515 Sources: GOC:pj Also known as: phytochrome chromophore anabolism, phytochrome chromophore biosynthesis, phytochrome chromophore formation, phytochrome chromophore synthesis Relationships: is a type of GO:0009058; is_a pigment biosynthetic process [GO:0046148]